{
  "term_id": "UNKNOWN:0002",
  "gene_name": "Coiled-coil domain-containing glutamate-rich protein 2",
  "term_label": "Unknown biological process",
  "gene": "UniProtKB:I3L3R5",
  "gene_symbol": "CCER2"
}